renal capsule development [GO:0072127] (BP) Relationships: is a type of connective tissue development [GO:0061448]; is part of kidney development [GO:0001822] Subtypes: mesonephric capsule development [GO:0061285], metanephric capsule development [GO:0072213] Definition: The process whose specific outcome is the progression of the renal capsule over time, from its formation to the mature structure. The renal capsule is the tough fibrous layer surrounding the kidney, covered in a thick layer of perinephric adipose tissue. It provides some protection from trauma and damage. During development, it comprises a single layer of flattened cells that lie just above the cortical stroma and the condensed mesenchyme of the nephrogenic zone. It is in this region that the early stages of nephron induction and formation of new generations ureteric bud branches occur, as the kidney expands. Sources: GOC:mtg_kidney_jan10